{
  "gene": "UniProtKB:Q8N5C1",
  "gene_name": "Calcium homeostasis modulator protein 5",
  "term_id": "GO:0005261",
  "gene_symbol": "CALHM5",
  "term_label": "monoatomic cation channel activity"
}